{
  "term_id": "GO:2000892",
  "term_label": "cellobiose catabolic process",
  "gene": "UniProtKB:P09848",
  "gene_symbol": "LCT",
  "gene_name": "Lactase_phlorizin hydrolase"
}